{
  "term_label": "U2 snRNA binding",
  "gene_name": "Coilin",
  "term_id": "GO:0030620",
  "gene_symbol": "COIL",
  "gene": "UniProtKB:P38432"
}